{
  "gene_name": "CCR4-NOT transcription complex subunit 7",
  "gene": "UniProtKB:Q9UIV1",
  "term_id": "GO:0004535",
  "gene_symbol": "CNOT7",
  "term_label": "poly(A)-specific ribonuclease activity"
}